NADP-malic enzyme C4 photosynthesis [GO:0009762] (BP) Definition: The process of C4 photosynthesis, as it occurs in plants in which the enzyme decarboxylating C4 acids in the bundle sheath is NADP-malic enzyme. Relationships: is a type of C4 photosynthesis [GO:0009760] References: PMID:11788762